{
  "gene": "UniProtKB:Q9UPX6",
  "term_label": "negative regulation of TOR signaling",
  "term_id": "GO:0032007",
  "gene_symbol": "MINAR1",
  "gene_name": "Major intrinsically disordered Notch2-binding receptor 1"
}